{
  "gene": "UniProtKB:O43304",
  "gene_symbol": "SEC14L5",
  "term_label": "Unknown biological process",
  "gene_name": "SEC14-like protein 5",
  "term_id": "UNKNOWN:0002"
}